{
  "gene": "UniProtKB:P49815",
  "term_id": "GO:0033596",
  "gene_symbol": "TSC2",
  "term_label": "TSC1-TSC2 complex",
  "gene_name": "Tuberin"
}